{
  "gene": "UniProtKB:Q16763",
  "gene_symbol": "UBE2S",
  "gene_name": "Ubiquitin-conjugating enzyme E2 S",
  "term_label": "ubiquitin-dependent protein catabolic process",
  "term_id": "GO:0006511"
}